{
  "gene_name": "Ecotropic viral integration site 5 protein homolog",
  "term_label": "retrograde transport, endosome to Golgi",
  "gene": "UniProtKB:O60447",
  "term_id": "GO:0042147",
  "gene_symbol": "EVI5"
}